{
  "term_id": "GO:0045087",
  "term_label": "innate immune response",
  "gene_symbol": "TRIM38",
  "gene": "UniProtKB:O00635",
  "gene_name": "E3 ubiquitin-protein ligase TRIM38"
}